{
  "gene_symbol": "CYP2J2",
  "gene_name": "Cytochrome P450 2J2",
  "term_label": "cytoplasm",
  "gene": "UniProtKB:P51589",
  "term_id": "GO:0005737"
}